{
  "gene_name": "Asc-type amino acid transporter 1",
  "term_label": "D-serine transmembrane transport",
  "gene": "UniProtKB:Q9NS82",
  "gene_symbol": "SLC7A10",
  "term_id": "GO:0042942"
}